{
  "term_label": "protein auto-ADP-ribosylation",
  "gene_name": "Protein mono-ADP-ribosyltransferase PARP12",
  "gene": "UniProtKB:Q9H0J9",
  "gene_symbol": "PARP12",
  "term_id": "GO:0070213"
}